regulation of lateral motor column neuron migration [GO:1902076] (BP) Definition: Any process that modulates the frequency, rate or extent of lateral motor column neuron migration. References: PMID:20711475 Sources: GOC:TermGenie, GOC:yaf Subtypes: negative regulation of lateral motor column neuron migration [GO:1902077], positive regulation of lateral motor column neuron migration [GO:1902078] Relationships: is a type of regulation of motor neuron migration [GO:1905483]; regulates lateral motor column neuron migration [GO:0097477]